negative regulation of platelet-derived growth factor receptor-beta signaling pathway [GO:2000587] (biological process) Also known as: negative regulation of PDGF receptor-beta signaling pathway, negative regulation of PDGFR-beta signaling pathway, negative regulation of betaPDGF receptor signaling pathway, negative regulation of platelet-derived growth factor receptor-beta signalling pathway Sources: GOC:obol Relationships: is a type of negative regulation of platelet-derived growth factor receptor signaling pathway [GO:0010642]; is a type of regulation of platelet-derived growth factor receptor-beta signaling pathway [GO:2000586]; negatively regulates platelet-derived growth factor receptor-beta signaling pathway [GO:0035791] Definition: Any process that stops, prevents or reduces the frequency, rate or extent of platelet-derived growth factor receptor-beta signaling pathway.